regulation of membrane depolarization [GO:0003254] (biological process) Definition: Any process that modulates the rate, frequency or extent of membrane depolarization. Membrane depolarization is the process in which membrane potential changes in the depolarizing direction from the resting potential, usually from negative to positive. Sources: GOC:dph, GOC:tb Relationships: is_a regulation of membrane potential [GO:0042391]; is a type of regulation of cellular process [GO:0050794]; regulates membrane depolarization [GO:0051899] Subtypes: regulation of mitochondrial depolarization [GO:0051900], GO:0060371, regulation of ventricular cardiac muscle cell membrane depolarization [GO:0060373], regulation of membrane depolarization during action potential [GO:0098902], negative regulation of membrane depolarization [GO:1904180], GO:1904181